origin recognition complex [GO:0000808] (cellular component) Relationships: is_a GO:0032991; is part of GO:0005694 Sources: GOC:elh Definition: A multisubunit complex that is located at the replication origins of a chromosome. Also known as: ORC, origin of replication recognition complex Subtypes: cytoplasmic origin of replication recognition complex [GO:0000809], nuclear origin of replication recognition complex [GO:0005664]